{
  "term_label": "Unknown molecular function",
  "gene": "UniProtKB:A6NLE4",
  "gene_symbol": "SMIM23",
  "term_id": "UNKNOWN:0001",
  "gene_name": "Small integral membrane protein 23"
}